{
  "gene_symbol": "C1orf100",
  "term_id": "UNKNOWN:0002",
  "gene_name": "Uncharacterized protein C1orf100",
  "term_label": "Unknown biological process",
  "gene": "UniProtKB:Q5SVJ3"
}